negative regulation of Schwann cell migration [GO:1900148] (biological process) Subtypes: GO:1904267 Sources: GOC:TermGenie, GOC:sjw Also known as: down regulation of Schwann cell migration, down-regulation of Schwann cell migration, downregulation of Schwann cell migration, inhibition of Schwann cell migration Relationships: is a type of regulation of Schwann cell migration [GO:1900147]; is a type of negative regulation of glial cell migration [GO:1903976]; negatively regulates Schwann cell migration [GO:0036135] Definition: Any process that stops, prevents or reduces the frequency, rate or extent of Schwann cell migration.